{
  "term_id": "GO:0140575",
  "gene_name": "Transmembrane reductase CYB561D2",
  "term_label": "transmembrane monodehydroascorbate reductase activity",
  "gene_symbol": "CYB561D2",
  "gene": "UniProtKB:O14569"
}